{
  "term_id": "GO:0006357",
  "term_label": "regulation of transcription by RNA polymerase II",
  "gene_symbol": "LHX2",
  "gene": "UniProtKB:P50458",
  "gene_name": "LIM_homeobox protein Lhx2"
}